{
  "gene": "UniProtKB:Q52WX2",
  "gene_symbol": "SBK1",
  "gene_name": "Serine_threonine-protein kinase SBK1",
  "term_id": "GO:0004674",
  "term_label": "protein serine/threonine kinase activity"
}